lymphatic endothelial cell differentiation [GO:0060836] (biological process) Sources: GOC:dph, GOC:sdb_2009, GOC:tb Relationships: is a type of GO:0045446; is part of lymph vessel development [GO:0001945] Definition: The process in which a venous blood vessel endothelial cell acquires specialized features of a lymphatic vessel endothelial cell, a thin flattened cell that lines the inside surfaces of lymph vessels.